{
  "gene_name": "Probable E3 ubiquitin-protein ligase MID2",
  "term_id": "GO:0008017",
  "term_label": "microtubule binding",
  "gene": "UniProtKB:Q9UJV3",
  "gene_symbol": "MID2"
}